{
  "gene": "UniProtKB:P01877",
  "gene_symbol": "IGHA2",
  "term_id": "GO:0006958",
  "term_label": "complement activation, classical pathway",
  "gene_name": "Immunoglobulin heavy constant alpha 2"
}